{
  "term_label": "regulation of cell population proliferation",
  "gene": "UniProtKB:P42229",
  "gene_symbol": "STAT5A",
  "gene_name": "Signal transducer and activator of transcription 5A",
  "term_id": "GO:0042127"
}